{
  "term_label": "Unknown cellular component",
  "term_id": "UNKNOWN:0003",
  "gene": "UniProtKB:A0A075B6U7",
  "gene_name": "T cell receptor alpha joining 23 (Fragment)",
  "gene_symbol": "TRAJ23"
}